bromoxynil metabolic process [GO:0018881] (biological process) Relationships: is a type of phenol-containing compound metabolic process [GO:0018958]; is a type of GO:0042537; is a type of GO:0050898; is a type of organohalogen metabolic process [GO:0090345] Also known as: bromoxynil metabolism Definition: The chemical reactions and pathways involving bromoxynil, C7H3Br2NO, a dibrominated phenol derivative with a cyano (-CN) group attached. Bromoxynil is used as a herbicide for post-emergent control of annual broadleaf weeds and works by inhibiting photosynthesis in the target plants. Sources: GOC:ai